{
  "gene_name": "Large neutral amino acids transporter small subunit 2",
  "gene": "UniProtKB:Q9UHI5",
  "gene_symbol": "SLC7A8",
  "term_id": "GO:0003333",
  "term_label": "amino acid transmembrane transport"
}